{
  "term_label": "endocytic recycling",
  "gene_symbol": "WASH6P",
  "term_id": "GO:0032456",
  "gene": "UniProtKB:Q9NQA3",
  "gene_name": "WAS protein family homolog 6"
}